centrosome cycle [GO:0007098] (biological process) Definition: The cell cycle process in which centrosome duplication and separation takes place. The centrosome cycle can operate with a considerable degree of independence from other processes of the cell cycle. Sources: ISBN:0815316194 Also known as: centrosome organisation, centrosome organization, centrosome organization and biogenesis Relationships: is a type of cell cycle process [GO:0022402]; is a type of microtubule organizing center organization [GO:0031023] Regulation: RO_0002211 by regulation of centrosome cycle [GO:0046605]; negatively regulated by GO:0046606; positively regulated by positive regulation of centrosome cycle [GO:0046607]